{
  "gene": "UniProtKB:Q9C0C4",
  "term_id": "GO:0030335",
  "gene_name": "Semaphorin-4C",
  "gene_symbol": "SEMA4C",
  "term_label": "positive regulation of cell migration"
}